{
  "gene": "UniProtKB:P04921",
  "term_label": "membrane",
  "term_id": "GO:0016020",
  "gene_symbol": "GYPC",
  "gene_name": "Glycophorin-C"
}